{
  "gene": "UniProtKB:Q7L1S5",
  "gene_name": "Carbohydrate sulfotransferase 9",
  "term_id": "UNKNOWN:0003",
  "term_label": "Unknown cellular component",
  "gene_symbol": "CHST9"
}